{
  "term_label": "calcium ion transmembrane transport",
  "term_id": "GO:0070588",
  "gene": "UniProtKB:P56373",
  "gene_symbol": "P2RX3",
  "gene_name": "P2X purinoceptor 3"
}